{
  "gene": "UniProtKB:P0DPA2",
  "term_label": "Unknown molecular function",
  "gene_name": "V-set and immunoglobulin domain-containing protein 8",
  "term_id": "UNKNOWN:0001",
  "gene_symbol": "VSIG8"
}